siRNA processing [GO:0030422] (biological process) Definition: A process leading to the generation of a functional small interfering RNA (siRNA). Includes the cleavage of double-stranded RNA to form small interfering RNA molecules (siRNAs) of 21-23 nucleotides. May also include amplification of the siRNA by RNA-directed RNA polymerase. Subtypes: GO:0010267, lsiRNA processing [GO:0010599] References: PMID:11524674, PMID:19239886, PMID:20687832 Sources: GOC:mah Regulation: regulated by GO:0070921; negatively regulated by negative regulation of siRNA processing [GO:1903704]; positively regulated by positive regulation of siRNA processing [GO:1903705] Also known as: RNA interference, production of guide RNAs, RNA interference, production of siRNA, chromatin silencing by small RNA, production of guide RNAs, chromatin silencing by small RNA, production of siRNA, production of guide RNAs involved in RNA interference, production of guide RNAs involved in chromatin silencing by small RNA, production of siRNA involved in RNA interference, production of siRNA involved in chromatin silencing by small RNA, production of siRNA involved in post-transcriptional gene silencing by RNA, production of siRNA involved in gene silencing by small RNA, production of siRNA, production of siRNA involved in PTGS Relationships: is_a regulatory ncRNA processing [GO:0070918]